{
  "gene_name": "Plakophilin-2",
  "term_id": "GO:0005886",
  "gene_symbol": "PKP2",
  "term_label": "plasma membrane",
  "gene": "UniProtKB:Q99959"
}